regulation of translational initiation in response to osmotic stress [GO:0043561] (biological process) Sources: GOC:dph, GOC:jl, GOC:tb Relationships: is a type of regulation of translation in response to osmotic stress [GO:0043557]; is a type of regulation of translational initiation in response to stress [GO:0043558] Subtypes: negative regulation of translational initiation in response to osmotic stress [GO:0032063], GO:0032064 Definition: Any process that modulates the frequency, rate or extent of translation initiation, as a result of a stimulus indicating an increase or decrease in the concentration of solutes outside the organism or cell.